aryldialkylphosphatase activity [GO:0004063] (molecular function) Definition: Catalysis of the reaction: aryl dialkyl phosphate + H2O = dialkyl phosphate + an aryl alcohol. Also known as: A-esterase activity, organophosphate esterase activity, organophosphate hydrolase activity, organophosphorus acid anhydrase activity, organophosphorus hydrolase activity, paraoxon hydrolase activity, paraoxonase activity, aryltriphosphate dialkylphosphohydrolase activity, paraoxon esterase activity, phosphotriesterase activity, pirimiphos-methyloxon esterase activity, OPH, aryltriphosphatase activity, esterase B1, esterase E4 Relationships: is a type of phosphoric triester hydrolase activity [GO:0016795] Sources: EC:3.1.8.1